aspartate ammonia-lyase activity [GO:0008797] (molecular function) Relationships: is a type of ammonia-lyase activity [GO:0016841] Also known as: L-aspartase activity, L-aspartate ammonia-lyase (fumarate-forming), L-aspartate ammonia-lyase activity, aspartase activity, fumaric aminase activity Definition: Catalysis of the reaction: L-aspartate = fumarate + NH3. Sources: EC:4.3.1.1